{
  "gene_symbol": "PI4K2B",
  "term_id": "GO:0007032",
  "term_label": "endosome organization",
  "gene_name": "Phosphatidylinositol 4-kinase type 2-beta",
  "gene": "UniProtKB:Q8TCG2"
}